{
  "gene_name": "E3 ubiquitin-protein ligase UBR5",
  "gene": "UniProtKB:O95071",
  "term_label": "cytoplasm",
  "gene_symbol": "UBR5",
  "term_id": "GO:0005737"
}